{
  "gene_symbol": "CEP95",
  "term_id": "UNKNOWN:0002",
  "gene_name": "Centrosomal protein of 95 kDa",
  "term_label": "Unknown biological process",
  "gene": "UniProtKB:Q96GE4"
}